{
  "term_label": "nucleus",
  "gene": "UniProtKB:O75995",
  "term_id": "GO:0005634",
  "gene_symbol": "SASH3",
  "gene_name": "SAM and SH3 domain-containing protein 3"
}